atrial cardiac muscle cell differentiation [GO:0055011] (biological process) Relationships: is_a cardiac muscle cell differentiation [GO:0055007] Also known as: atrial cardiomyocyte differentiation, atrial heart muscle cell differentiation Definition: The process in which a relatively unspecialized cell acquires specialized features of a cardiac muscle cell in the atrium. Cardiac muscle cells are striated muscle cells that are responsible for heart contraction. The atrium is the part of the heart that receives blood into the organ. Sources: GOC:devbiol, GOC:mtg_heart